{
  "gene_symbol": "SNX16",
  "term_id": "GO:0001881",
  "term_label": "receptor recycling",
  "gene": "UniProtKB:P57768",
  "gene_name": "Sorting nexin-16"
}